{
  "term_label": "calcium sensitive guanylate cyclase activator activity",
  "gene_symbol": "GUCA1B",
  "gene": "UniProtKB:Q9UMX6",
  "term_id": "GO:0008048",
  "gene_name": "Guanylyl cyclase-activating protein 2"
}